piperidine N-piperoyltransferase activity [GO:0050199] (MF) Sources: EC:2.3.1.145, RHEA:14561 Relationships: is a type of acyltransferase activity, transferring groups other than amino-acyl groups [GO:0016747] Also known as: (E,E)-piperoyl-CoA:piperidine N-piperoyltransferase activity, piperidine piperoyltransferase activity, piperoyl-CoA:piperidine N-piperoyltransferase activity Definition: Catalysis of the reaction: (E,E)-piperoyl-CoA + piperidine = N-[(E,E)-piperoyl]piperidine + CoA + H+.